cytoskeleton organization [GO:0007010] (biological process) Definition: A process that is carried out at the cellular level which results in the assembly, arrangement of constituent parts, or disassembly of cytoskeletal structures. Sources: GOC:dph, GOC:jl, GOC:mah Also known as: cytoskeleton organisation, cytoskeletal organization and biogenesis, cytoskeletal regulator activity, cytoskeleton organization and biogenesis Relationships: is_a organelle organization [GO:0006996] Subtypes: microtubule cytoskeleton organization [GO:0000226], actin cytoskeleton organization [GO:0030036], GO:0030865, establishment or maintenance of cytoskeleton polarity [GO:0030952], septin cytoskeleton organization [GO:0032185], intermediate filament cytoskeleton organization [GO:0045104], cytoskeletal rearrangement involved in phagocytosis, engulfment [GO:0060097], GO:0099187, postsynaptic cytoskeleton organization [GO:0099188] Regulation: regulated by regulation of cytoskeleton organization [GO:0051493]; negatively regulated by negative regulation of cytoskeleton organization [GO:0051494]; positively regulated by positive regulation of cytoskeleton organization [GO:0051495]